cholesterol O-acyltransferase activity [GO:0034736] (molecular function) Relationships: is a type of sterol O-acyltransferase activity [GO:0004772] Definition: Catalysis of the reaction: acyl-CoA + cholesterol = a cholesterol ester + CoA. Also known as: ACAT activity, cholesterol acyltransferase activity, acylcoenzyme A:cholesterol O-acyltransferase activity, acyl coenzyme A-cholesterol-O-acyltransferase activity, acyl-CoA:cholesterol O-acyltransferase activity, acyl-CoA:cholesterol acyltransferase activity, cholesterol ester synthetase activity, cholesteryl ester synthetase activity Sources: RHEA:17729